{
  "gene_name": "Testis-specific Y-encoded-like protein 1",
  "gene_symbol": "TSPYL1",
  "gene": "UniProtKB:Q9H0U9",
  "term_id": "GO:0005634",
  "term_label": "nucleus"
}